{
  "gene": "UniProtKB:Q6ICL3",
  "gene_name": "Transport and Golgi organization protein 2 homolog",
  "term_label": "protein secretion",
  "term_id": "GO:0009306",
  "gene_symbol": "TANGO2"
}